{
  "gene_symbol": "QDPR",
  "term_label": "6,7-dihydropteridine reductase activity",
  "gene_name": "Dihydropteridine reductase",
  "gene": "UniProtKB:P09417",
  "term_id": "GO:0004155"
}